{
  "term_id": "GO:0007064",
  "gene": "UniProtKB:Q96FF9",
  "gene_name": "Sororin",
  "gene_symbol": "CDCA5",
  "term_label": "mitotic sister chromatid cohesion"
}